response to tetralin [GO:1901498] (biological process) Sources: GOC:TermGenie, GOC:mengo_curators Relationships: is a type of response to chemical [GO:0042221] Definition: Any process that results in a change in state or activity of a cell or an organism (in terms of movement, secretion, enzyme production, gene expression, etc.) as a result of a tetralin stimulus.